{
  "gene_symbol": "RP1L1",
  "term_label": "photoreceptor cell outer segment organization",
  "term_id": "GO:0035845",
  "gene_name": "Retinitis pigmentosa 1-like 1 protein",
  "gene": "UniProtKB:Q8IWN7"
}